regulation of secondary metabolic process [GO:0043455] (biological process) Sources: GOC:jl Definition: Any process that modulates the frequency, rate or extent of secondary metabolism, the chemical reactions and pathways involving compounds that are not necessarily required for growth and maintenance of cells, and are often unique to a taxon. Relationships: is a type of regulation of metabolic process [GO:0019222]; regulates GO:0019748 Also known as: regulation of secondary metabolism Subtypes: regulation of gibberellin biosynthetic process [GO:0010371], positive regulation of penicillin metabolic process [GO:0033246], regulation of penicillin catabolic process [GO:0033247], regulation of melanization defense response [GO:0035007], GO:1900376, regulation of fumagillin biosynthetic process [GO:1902090], GO:2000762